{
  "term_id": "GO:0007165",
  "gene_name": "V-set and transmembrane domain-containing protein 1",
  "term_label": "signal transduction",
  "gene_symbol": "VSTM1",
  "gene": "UniProtKB:Q6UX27"
}